{
  "term_label": "mitochondrion",
  "term_id": "GO:0005739",
  "gene_symbol": "PPM1J",
  "gene_name": "Protein phosphatase 1J",
  "gene": "UniProtKB:Q5JR12"
}